{
  "gene": "UniProtKB:P43652",
  "gene_symbol": "AFM",
  "term_label": "Unknown cellular component",
  "gene_name": "Afamin",
  "term_id": "UNKNOWN:0003"
}